{
  "term_label": "oligosaccharide binding",
  "gene_name": "Chitinase domain-containing protein 1",
  "gene_symbol": "CHID1",
  "term_id": "GO:0070492",
  "gene": "UniProtKB:Q9BWS9"
}